{
  "gene_symbol": "ADAMTSL3",
  "term_id": "UNKNOWN:0001",
  "term_label": "Unknown molecular function",
  "gene": "UniProtKB:P82987",
  "gene_name": "ADAMTS-like protein 3"
}